{
  "term_id": "GO:0005172",
  "gene": "UniProtKB:P49765",
  "term_label": "vascular endothelial growth factor receptor binding",
  "gene_name": "Vascular endothelial growth factor B",
  "gene_symbol": "VEGFB"
}